regulation of centrosome duplication [GO:0010824] (biological process) Sources: GOC:dph, GOC:tb Subtypes: positive regulation of centrosome duplication [GO:0010825], negative regulation of centrosome duplication [GO:0010826], regulation of centriole replication [GO:0046599] Definition: Any process that modulates the frequency, rate or extent of centrosome duplication. Centrosome duplication is the replication of a centrosome, a structure comprised of a pair of centrioles and peri-centriolar material from which a microtubule spindle apparatus is organized. Relationships: is_a GO:0046605; regulates centrosome duplication [GO:0051298]